{
  "term_label": "membrane",
  "term_id": "GO:0016020",
  "gene_name": "Olfactory receptor 10J4",
  "gene": "UniProtKB:P0C629",
  "gene_symbol": "OR10J4"
}